protein localization to meiotic spindle pole body [GO:1902441] (biological process) References: PMID:20833892 Relationships: is_a protein localization to spindle pole body [GO:0071988]; is part of meiotic spindle pole body organization [GO:1990395] Regulation: regulated by regulation of protein localization to meiotic spindle pole body [GO:0140433]; positively regulated by positive regulation of protein localization to meiotic spindle pole body [GO:0140434]; RO_0002212 by negative regulation of protein localization to meiotic spindle pole body [GO:0140435] Also known as: protein localisation in meiotic spindle pole body, protein localisation to meiotic spindle pole body, protein localization in meiotic spindle pole body, protein location to meiotic spindle pole body, establishment of protein localization to meiotic spindle pole body Definition: A process in which a protein is transported to, or maintained in, a location within a meiotic spindle pole body.